{
  "term_label": "plasma membrane",
  "gene_name": "Potassium channel subfamily K member 7",
  "term_id": "GO:0005886",
  "gene": "UniProtKB:Q9Y2U2",
  "gene_symbol": "KCNK7"
}